L-methionine:2-oxoglutarate aminotransferase activity [GO:0080099] (molecular function) Definition: Catalysis of the reaction: L-methionine + 2-oxoglutarate = 4-methylthio-2-oxobutyrate + L-glutamate. References: PMID:18394996 Also known as: L-methionine:alpha-ketoglutarate aminotransferase activity Note: This reaction falls within the larger set of reactions associated with EC:2.6.1.5 (See BRENDA: http://www.brenda-enzymes.org/php/result_flat.php4?ecno=2.6.1.5). Relationships: is a type of methionine-oxo-acid transaminase activity [GO:0010326]